{
  "term_id": "GO:0002250",
  "gene_symbol": "IFNA2",
  "gene": "UniProtKB:P01563",
  "term_label": "adaptive immune response",
  "gene_name": "Interferon alpha-2"
}